{
  "gene": "UniProtKB:Q86VH2",
  "term_label": "cytoplasm",
  "term_id": "GO:0005737",
  "gene_symbol": "KIF27",
  "gene_name": "Kinesin-like protein KIF27"
}